{
  "term_id": "GO:0050728",
  "gene_symbol": "TNFAIP8L2",
  "gene": "UniProtKB:Q6P589",
  "term_label": "negative regulation of inflammatory response",
  "gene_name": "Tumor necrosis factor alpha-induced protein 8-like protein 2"
}